{
  "term_id": "GO:0031012",
  "gene_symbol": "DMBT1",
  "gene": "UniProtKB:Q9UGM3",
  "gene_name": "Deleted in malignant brain tumors 1 protein",
  "term_label": "extracellular matrix"
}